{
  "term_id": "GO:0007099",
  "gene_symbol": "CCDC57",
  "gene": "UniProtKB:Q2TAC2",
  "gene_name": "Coiled-coil domain-containing protein 57",
  "term_label": "centriole replication"
}